{
  "term_label": "ubiquitin protein ligase activity",
  "gene": "UniProtKB:Q9UBF6",
  "gene_name": "RING-box protein 2",
  "term_id": "GO:0061630",
  "gene_symbol": "RNF7"
}